{
  "gene_symbol": "CAT",
  "gene_name": "Catalase",
  "term_id": "GO:0005739",
  "gene": "UniProtKB:P04040",
  "term_label": "mitochondrion"
}